regulation of hippocampal neuron apoptotic process [GO:0110089] (biological process) Subtypes: positive regulation of hippocampal neuron apoptotic process [GO:0110090], negative regulation of hippocampal neuron apoptotic process [GO:0110091] Definition: Any process that modulates the occurrence or rate of cell death by apoptotic process in hippocampal neurons. Relationships: is a type of GO:0043523; regulates hippocampal neuron apoptotic process [GO:0110088] References: PMID:18940801 Sources: GOC:sl